protein alkylation [GO:0008213] (biological process) Definition: The addition of an alkyl group to a protein amino acid. Alkyl groups are derived from alkanes by removal of one hydrogen atom. Sources: GOC:ma Also known as: protein amino acid alkylation Relationships: is a type of protein modification process [GO:0036211] Subtypes: GO:0006479